{
  "gene_symbol": "CXCR3",
  "term_label": "calcium-mediated signaling",
  "term_id": "GO:0019722",
  "gene": "UniProtKB:P49682",
  "gene_name": "C-X-C chemokine receptor type 3"
}